carbohydrate kinase activity [GO:0019200] (molecular function) Sources: GOC:jl Subtypes: GO:0004335, hexokinase activity [GO:0004396], ketohexokinase activity [GO:0004454], ribokinase activity [GO:0004747], D-xylulokinase activity [GO:0004856], phosphofructokinase activity [GO:0008443], GO:0008671, GO:0008673, GO:0008737, ribulokinase activity [GO:0008741], GO:0008744, GO:0008993, GO:0009384, GO:0009702, D-ribulokinase activity [GO:0019150], heptose 7-phosphate kinase activity [GO:0033785], N-acetylgalactosamine kinase activity [GO:0033858], ribose 1,5-bisphosphate phosphokinase activity [GO:0033863], N-acetylglucosamine kinase activity [GO:0045127] Relationships: is a type of kinase activity [GO:0016301]; is part of carbohydrate phosphorylation [GO:0046835] Definition: Catalysis of the transfer of a phosphate group, usually from ATP, to a carbohydrate substrate molecule.